{
  "term_id": "UNKNOWN:0001",
  "gene": "UniProtKB:Q9H7P6",
  "term_label": "Unknown molecular function",
  "gene_name": "Multivesicular body subunit 12B",
  "gene_symbol": "MVB12B"
}